{
  "gene_symbol": "DACT1",
  "term_label": "Unknown molecular function",
  "gene": "UniProtKB:Q9NYF0",
  "term_id": "UNKNOWN:0001",
  "gene_name": "Dapper homolog 1"
}